{
  "gene_name": "Humanin-like 6",
  "term_id": "GO:1900118",
  "gene": "UniProtKB:P0CJ73",
  "term_label": "negative regulation of execution phase of apoptosis",
  "gene_symbol": "MTRNR2L6"
}